{
  "gene_symbol": "TRAPPC13",
  "term_id": "GO:1990072",
  "gene": "UniProtKB:A5PLN9",
  "term_label": "TRAPPIII protein complex",
  "gene_name": "Trafficking protein particle complex subunit 13"
}